{
  "term_label": "Unknown cellular component",
  "gene_symbol": "CAPZB",
  "gene": "UniProtKB:P47756",
  "term_id": "UNKNOWN:0003",
  "gene_name": "F-actin-capping protein subunit beta"
}